{
  "term_id": "UNKNOWN:0001",
  "term_label": "Unknown molecular function",
  "gene": "UniProtKB:Q9H2G9",
  "gene_name": "Golgin-45",
  "gene_symbol": "BLZF1"
}